{
  "term_id": "GO:0007342",
  "gene": "UniProtKB:P15328",
  "term_label": "fusion of sperm to egg plasma membrane involved in single fertilization",
  "gene_symbol": "FOLR1",
  "gene_name": "Folate receptor alpha"
}